multiple spine synapse organization, multiple dendrites [GO:0150091] (biological process) Relationships: is a type of multiple spine synapse organization [GO:0150089] Definition: A process that is carried out at the cellular level which results in the assembly, arrangement of constituent parts, or disassembly of a synapse between a multiple synapse bouton and two or more dendritic spines protruding either from a single dendrite or from multiple dendrites. References: PMID:10586883, PMID:11248111, PMID:22028887, PMID:24487234, PMID:7482800, PMID:8366344 Sources: GOC:aruk, GOC:bc